regulation of skeletal muscle contraction by modulation of calcium ion sensitivity of myofibril [GO:0014723] (biological process) Relationships: is a type of regulation of skeletal muscle contraction by calcium ion signaling [GO:0014722] Also known as: regulation of calcium ion sensitivity of myofibril involved in skeletal muscle contraction Sources: GOC:mtg_muscle Definition: Any process that modulates the frequency, rate or extent of skeletal muscle contraction by changing calcium ion binding affinity of the myofibril.